negative regulation of extrathymic T cell differentiation [GO:0033086] (biological process) Relationships: is a type of regulation of extrathymic T cell differentiation [GO:0033082]; is a type of GO:0045581; RO_0002212 extrathymic T cell differentiation [GO:0033078] Also known as: negative regulation of extrathymic T cell development Note: Note that immunologists typically use the word 'development' to refer to cells of B or T cell lineages undergoing the process that GO describes as 'cell differentiation'. Sources: GOC:add, GOC:mah Definition: Any process that stops, prevents, or reduces the frequency, rate or extent of extrathymic T cell differentiation.